{
  "gene_symbol": "POLR3GL",
  "gene": "UniProtKB:Q9BT43",
  "gene_name": "DNA-directed RNA polymerase III subunit RPC7-like",
  "term_id": "GO:0005666",
  "term_label": "RNA polymerase III complex"
}